{
  "term_id": "UNKNOWN:0001",
  "gene_name": "Ankyrin repeat domain-containing protein 16",
  "term_label": "Unknown molecular function",
  "gene_symbol": "ANKRD16",
  "gene": "UniProtKB:Q6P6B7"
}